{
  "gene_symbol": "FUT1",
  "gene_name": "Galactoside alpha-(1,2)-fucosyltransferase 1",
  "term_label": "Unknown biological process",
  "gene": "UniProtKB:P19526",
  "term_id": "UNKNOWN:0002"
}